{
  "term_label": "Unknown molecular function",
  "gene_symbol": "DNAAF8",
  "gene": "UniProtKB:Q8IYS4",
  "term_id": "UNKNOWN:0001",
  "gene_name": "Dynein axonemal assembly factor 8"
}